{
  "term_id": "GO:0042632",
  "gene_symbol": "APOA2",
  "gene_name": "Apolipoprotein A-II",
  "term_label": "cholesterol homeostasis",
  "gene": "UniProtKB:P02652"
}